{
  "gene_symbol": "GCSAM",
  "gene": "UniProtKB:Q8N6F7",
  "gene_name": "Germinal center-associated signaling and motility protein",
  "term_id": "UNKNOWN:0001",
  "term_label": "Unknown molecular function"
}